{
  "gene": "UniProtKB:Q96NU0",
  "gene_symbol": "CNTNAP3B",
  "term_id": "GO:0007399",
  "term_label": "nervous system development",
  "gene_name": "Contactin-associated protein-like 3B"
}